{
  "gene": "UniProtKB:P48048",
  "term_label": "plasma membrane",
  "gene_name": "ATP-sensitive inward rectifier potassium channel 1",
  "gene_symbol": "KCNJ1",
  "term_id": "GO:0005886"
}